procollagen galactosyltransferase activity [GO:0050211] (molecular function) Definition: Catalysis of the reaction: UDP-galactose + procollagen 5-hydroxy-L-lysine = UDP + procollagen 5-(D-galactosyloxy)-L-lysine. Also known as: UDP galactose-collagen galactosyltransferase activity, UDP-galactose:procollagen-5-hydroxy-L-lysine D-galactosyltransferase activity, UDPgalactose:5-hydroxylysine-collagen galactosyltransferase activity, UDPgalactose:procollagen-5-hydroxy-L-lysine D-galactosyltransferase activity, collagen galactosyltransferase activity, collagen hydroxylysyl galactosyltransferase activity, hydroxylysine galactosyltransferase activity, uridine diphosphogalactose-collagen galactosyltransferase activity Relationships: is a type of UDP-galactosyltransferase activity [GO:0035250]; is a type of catalytic activity, acting on a protein [GO:0140096] Sources: EC:2.4.1.50, MetaCyc:PROCOLLAGEN-GALACTOSYLTRANSFERASE-RXN